{
  "gene_name": "Olfactory receptor 2M7",
  "term_label": "plasma membrane",
  "gene": "UniProtKB:Q8NG81",
  "gene_symbol": "OR2M7",
  "term_id": "GO:0005886"
}